{
  "gene_symbol": "KLRC4",
  "term_label": "plasma membrane",
  "gene": "UniProtKB:O43908",
  "term_id": "GO:0005886",
  "gene_name": "NKG2-F type II integral membrane protein"
}